{
  "gene_name": "C-type lectin domain family 2 member D",
  "gene_symbol": "CLEC2D",
  "term_label": "external side of plasma membrane",
  "term_id": "GO:0009897",
  "gene": "UniProtKB:Q9UHP7"
}